endochondral bone growth [GO:0003416] (biological process) Definition: The increase in size or mass of an endochondral bone that contributes to the shaping of the bone. Relationships: is a type of bone growth [GO:0098868] Sources: GOC:ascb_2009, GOC:dph, GOC:tb